{
  "gene": "UniProtKB:P48960",
  "term_id": "GO:0007186",
  "term_label": "G protein-coupled receptor signaling pathway",
  "gene_symbol": "ADGRE5",
  "gene_name": "Adhesion G protein-coupled receptor E5"
}